muscle cell projection membrane [GO:0036195] (cellular component) Relationships: is a type of GO:0031253; BFO_0000050 muscle cell projection [GO:0036194] References: PMID:15930100, PMID:22464329 Sources: CL:0000187, GOC:kmv Definition: The portion of the plasma membrane surrounding a muscle cell projection.